polysaccharide biosynthetic process [GO:0000271] (biological process) Definition: The chemical reactions and pathways resulting in the formation of a polysaccharide, a polymer of many (typically more than 10) monosaccharide residues linked glycosidically. Sources: GOC:go_curators Also known as: glycan biosynthesis, glycan biosynthetic process, polysaccharide anabolism, polysaccharide biosynthesis, polysaccharide formation, polysaccharide synthesis Relationships: is_a polysaccharide metabolic process [GO:0005976]; is a type of macromolecule biosynthetic process [GO:0009059]; is a type of carbohydrate biosynthetic process [GO:0016051] Subtypes: lipopolysaccharide biosynthetic process [GO:0009103], O antigen biosynthetic process [GO:0009243], GO:0009246, K antigen biosynthetic process [GO:0009248], GO:0009250, fructan biosynthetic process [GO:0010146], Lewis a epitope biosynthetic process [GO:0010493], GO:0035884, alginic acid biosynthetic process [GO:0042121], GO:0045227, slime layer polysaccharide biosynthetic process [GO:0045228], pectin biosynthetic process [GO:0045489], galactomannan biosynthetic process [GO:0051070], 4,6-pyruvylated galactose residue biosynthetic process [GO:0051072], cell wall polysaccharide biosynthetic process [GO:0070592], mannogen biosynthetic process [GO:0106304] Regulation: regulated by regulation of polysaccharide biosynthetic process [GO:0032885]